cinnamic acid ester metabolic process [GO:0009801] (biological process) Also known as: cinnamic acid ester metabolism Subtypes: cinnamic acid ester biosynthetic process [GO:0009802], cinnamic acid ester catabolic process [GO:0046282] Definition: The chemical reactions and pathways involving ester derivatives of cinnamic acid, phenylpropenoic acid. Relationships: is a type of phenylpropanoid metabolic process [GO:0009698]; is_a olefinic compound metabolic process [GO:0120254] Sources: GOC:lr, GOC:yl